{
  "gene_symbol": "TAS2R4",
  "term_id": "GO:0001580",
  "gene": "UniProtKB:Q9NYW5",
  "gene_name": "Taste receptor type 2 member 4",
  "term_label": "detection of chemical stimulus involved in sensory perception of bitter taste"
}